{
  "term_id": "GO:0014069",
  "term_label": "postsynaptic density",
  "gene_name": "Kalirin",
  "gene_symbol": "KALRN",
  "gene": "UniProtKB:O60229"
}